epigallocatechin 3-gallate binding [GO:0097247] (molecular function) Also known as: catechin gallate binding, EGCG binding Relationships: is a type of flavonoid binding [GO:0097243] References: PMID:21307292 Sources: GOC:sl Definition: Binding to epigallocatechin 3-gallate, a compound that is a gallic acid ester of a catechin.